{
  "gene_name": "EH domain-binding protein 1-like protein 1",
  "term_id": "GO:0030036",
  "gene_symbol": "EHBP1L1",
  "gene": "UniProtKB:Q8N3D4",
  "term_label": "actin cytoskeleton organization"
}